{
  "gene_symbol": "ZBTB48",
  "term_label": "Unknown cellular component",
  "gene": "UniProtKB:P10074",
  "term_id": "UNKNOWN:0003",
  "gene_name": "Telomere zinc finger-associated protein"
}